{
  "term_label": "Unknown molecular function",
  "gene_symbol": "ISLR",
  "gene": "UniProtKB:O14498",
  "term_id": "UNKNOWN:0001",
  "gene_name": "Immunoglobulin superfamily containing leucine-rich repeat protein"
}